halotropism [GO:0170002] (BP) Relationships: is a type of tropism [GO:0009606] Definition: A sodium-specific negative tropism that is crucial for surviving and thriving under high salinity. Also known as: root halotropism References: PMID:36243013